epidermal lamellar body [GO:0097209] (cellular component) Relationships: is a type of lamellar body [GO:0042599] Sources: GOC:cjm, Wikipedia:Lamellar_granule Definition: A specialized secretory organelle found in keratinocytes and involved in the formation of an impermeable, lipid-containing membrane that serves as a water barrier and is required for correct skin barrier function.